{
  "gene_symbol": "ERLIN2",
  "term_label": "endoplasmic reticulum membrane",
  "gene_name": "Erlin-2",
  "term_id": "GO:0005789",
  "gene": "UniProtKB:O94905"
}